regulation of hormone biosynthetic process [GO:0046885] (biological process) Definition: Any process that modulates the frequency, rate or extent of the chemical reactions and pathways resulting in the formation of hormones. Sources: GOC:ai Also known as: regulation of hormone anabolism, regulation of hormone biosynthesis, regulation of hormone formation, regulation of hormone synthesis Relationships: is_a regulation of biosynthetic process [GO:0009889]; is a type of regulation of hormone metabolic process [GO:0032350]; regulates hormone biosynthetic process [GO:0042446] Subtypes: regulation of juvenile hormone biosynthetic process [GO:0007557], regulation of auxin biosynthetic process [GO:0010600], negative regulation of hormone biosynthetic process [GO:0032353], GO:0046886, regulation of steroid hormone biosynthetic process [GO:0090030], GO:1904076, regulation of progesterone biosynthetic process [GO:2000182]